facultative heterochromatin formation [GO:0140718] (biological process) Note: Note that facultative heterochromatin can be reprogrammed, as opposed to constitutive heterochromatin which usually cannot be reprogrammed to a transcriptionally-competent state. Note also that facultative heterochromatin formation does not usually involve DNA methylation, while constitutive heterochromatin formation does. Subtypes: rDNA heterochromatin formation [GO:0000183], GO:1902794, siRNA-mediated facultative heterochromatin formation [GO:1902795] Also known as: fHC assembly, facultative heterochromatin assembly Definition: The compaction of chromatin into a conformation that is refractory to transcription but that can be converted to euchromatin and allow transcription in specific contexts. These can be temporal (e.g., developmental states or specific cell-cycle stages), spatial (e.g., nuclear localization changes from the center to the periphery or vice versa due to exogenous factors/signals), or parental/heritable (e.g., monoallelic gene expression). In metazoa, this involves the methylation of histone H3K27. References: PMID:17936700 Relationships: is a type of GO:0031507